{
  "term_label": "adrenomedullin receptor signaling pathway",
  "term_id": "GO:1990410",
  "gene": "UniProtKB:C9JUS6",
  "gene_symbol": "ADM5",
  "gene_name": "Putative adrenomedullin-5-like protein"
}